{
  "gene": "UniProtKB:Q9Y6Q1",
  "gene_name": "Calpain-6",
  "term_label": "cytoplasm",
  "term_id": "GO:0005737",
  "gene_symbol": "CAPN6"
}